{
  "gene_name": "Nicotinamide_nicotinic acid mononucleotide adenylyltransferase 2",
  "term_id": "GO:0005794",
  "gene_symbol": "NMNAT2",
  "term_label": "Golgi apparatus",
  "gene": "UniProtKB:Q9BZQ4"
}